{
  "term_label": "proteasome core complex, alpha-subunit complex",
  "gene_name": "Proteasome subunit alpha type-2",
  "gene": "UniProtKB:P25787",
  "gene_symbol": "PSMA2",
  "term_id": "GO:0019773"
}